positive regulation terrein biosynthetic process [GO:0140881] (biological process) Relationships: is a type of positive regulation of secondary metabolite biosynthetic process [GO:1900378]; is a type of positive regulation of alcohol biosynthetic process [GO:1902932]; positively regulates GO:0140880 References: PMID:24816227, PMID:25852654 Definition: Any process that increases the rate, frequency or extent of the chemical reactions and pathways resulting in the formation of the fungal metabolite terrein.